{
  "term_label": "microtubule",
  "gene": "UniProtKB:Q12756",
  "term_id": "GO:0005874",
  "gene_symbol": "KIF1A",
  "gene_name": "Kinesin-like protein KIF1A"
}